arthro-series glucosylceramide biosynthetic process [GO:0140269] (BP) Relationships: is a type of glycosphingolipid biosynthetic process [GO:0006688] Definition: The chemical reactions and pathways resulting in the formation of arthro-series glucosylceramides that begins with the synthesis of a tetrasaccharide core GalNAc-beta-1,4-GlcNAc-beta-1,3-Man-beta-1,4Glc-ceramide. This core can be further elongated with the sequential addition of various carbohydrate units. References: PMID:35536927